{
  "gene_symbol": "ACTN4",
  "term_label": "actin cytoskeleton organization",
  "gene": "UniProtKB:O43707",
  "gene_name": "Alpha-actinin-4",
  "term_id": "GO:0030036"
}